{
  "term_label": "Unknown molecular function",
  "gene_name": "Reprimo-like protein",
  "gene_symbol": "RPRML",
  "gene": "UniProtKB:Q8N4K4",
  "term_id": "UNKNOWN:0001"
}